{
  "term_id": "GO:0042393",
  "gene": "UniProtKB:Q9UHJ3",
  "gene_symbol": "SFMBT1",
  "gene_name": "Scm-like with four MBT domains protein 1",
  "term_label": "histone binding"
}